negative regulation of axonogenesis [GO:0050771] (BP) Relationships: is a type of GO:0010977; is a type of negative regulation of neurogenesis [GO:0050768]; is a type of regulation of axonogenesis [GO:0050770]; negatively regulates axonogenesis [GO:0007409] Subtypes: negative regulation of axon extension [GO:0030517], negative regulation of collateral sprouting [GO:0048671] Definition: Any process that stops, prevents, or reduces the frequency, rate or extent of axonogenesis. Also known as: down regulation of axonogenesis, down-regulation of axonogenesis, downregulation of axonogenesis, inhibition of axonogenesis Sources: GOC:ai